postsynaptic specialization of symmetric synapse [GO:0099629] (cellular component) References: PMID:18832033 Definition: A network of proteins within and adjacent to the postsynaptic membrane of a symmetric synapse, consisting of anchoring and scaffolding molecules, signaling enzymes and cytoskeletal components that spatially and functionally organize the neurotransmitter receptors at the synapse. This structure is not as thick or electron dense as the postsynaptic densities found in asymmetric synapses. Relationships: is_a postsynaptic specialization [GO:0099572]; is part of GO:0032280 Also known as: postsynaptic density of inhibitory synapse